{
  "term_id": "GO:0006357",
  "term_label": "regulation of transcription by RNA polymerase II",
  "gene_name": "Zinc finger protein 568",
  "gene": "UniProtKB:Q3ZCX4",
  "gene_symbol": "ZNF568"
}